magnesium protoporphyrin IX methyltransferase activity [GO:0046406] (molecular function) Also known as: magnesium-protoporphyrin O-methyltransferase activity, (-)-S-adenosyl-L-methionine:magnesium-protoporphyrin IX methyltransferase activity, Mg-protoporphyrin IX methyltransferase activity, S-adenosyl-L-methionine:Mg protoporphyrin methyltransferase activity, S-adenosyl-L-methionine:magnesium-protoporphyrin O-methyltransferase activity, S-adenosyl-L-methionine:magnesium-protoporphyrin-IX O-methyltransferase activity, S-adenosylmethionine-magnesium protoporphyrin methyltransferase activity, S-adenosylmethioninemagnesium protoporphyrin methyltransferase activity Definition: Catalysis of the reaction: Mg-protoporphyrin IX + S-adenosyl-L-methionine = Mg-protoporphyrin IX 13-monomethyl ester + S-adenosyl-L-homocysteine. Sources: RHEA:17809 Relationships: is a type of O-methyltransferase activity [GO:0008171]; is a type of S-adenosylmethionine-dependent methyltransferase activity [GO:0008757]